{
  "term_id": "GO:0000212",
  "gene_symbol": "KATNAL2",
  "gene": "UniProtKB:Q8IYT4",
  "term_label": "meiotic spindle organization",
  "gene_name": "Katanin p60 ATPase-containing subunit A-like 2"
}